{
  "gene_symbol": "ZNF688",
  "gene": "UniProtKB:P0C7X2",
  "term_label": "RNA polymerase II cis-regulatory region sequence-specific DNA binding",
  "term_id": "GO:0000978",
  "gene_name": "Zinc finger protein 688"
}